{
  "gene_symbol": "DTNA",
  "gene": "UniProtKB:Q9Y4J8",
  "term_label": "plasma membrane",
  "term_id": "GO:0005886",
  "gene_name": "Dystrobrevin alpha"
}